{
  "gene_symbol": "LRPPRC",
  "gene": "UniProtKB:P42704",
  "gene_name": "Leucine-rich PPR motif-containing protein, mitochondrial",
  "term_id": "GO:0003730",
  "term_label": "mRNA 3'-UTR binding"
}